orotidine-5'-phosphate decarboxylase activity [GO:0004590] (molecular function) Also known as: ODCase activity, OMP decarboxylase activity, OMP-DC, OMPdcase activity, UMP synthase activity, orotate decarboxylase activity, orotate monophosphate decarboxylase activity, orotic decarboxylase activity, orotidine 5'-phosphate decarboxylase activity, orotidine monophosphate decarboxylase activity, orotidine phosphate decarboxylase activity, orotidine-5'-monophosphate decarboxylase activity, orotidine-5'-phosphate carboxy-lyase (UMP-forming), orotidine-5'-phosphate carboxy-lyase activity, orotidylic acid decarboxylase activity, orotidylic decarboxylase activity, orotodylate decarboxylase activity, uridine 5'-monophosphate synthase activity Definition: Catalysis of the reaction: H+ + orotidine 5'-phosphate = CO2 + UMP. Sources: EC:4.1.1.23, RHEA:11596 Relationships: is a type of carboxy-lyase activity [GO:0016831]